{
  "gene_symbol": "REST",
  "gene": "UniProtKB:Q13127",
  "term_label": "transcription repressor complex",
  "gene_name": "RE1-silencing transcription factor",
  "term_id": "GO:0017053"
}